succinyl-CoA:(R)-citramalate CoA-transferase activity [GO:0043961] (molecular function) Relationships: is a type of CoA-transferase activity [GO:0008410] Definition: Catalysis of the reaction: succinyl-CoA + (R)-citramalate = succinate + (R)-citramalyl-CoA. References: PMID:17259315 Sources: GOC:jl Also known as: succinyl-CoA:(R)-citramalate CoA transferase activity, succinyl-CoA:R-citramalate CoA transferase, L-carnitine dehydratase/bile acid-inducible protein F